{
  "gene_name": "E3 ubiquitin-protein ligase ZNRF1",
  "gene_symbol": "ZNRF1",
  "gene": "UniProtKB:Q8ND25",
  "term_id": "GO:0005737",
  "term_label": "cytoplasm"
}